{
  "term_label": "ATP hydrolysis activity",
  "gene": "UniProtKB:Q9NU22",
  "term_id": "GO:0016887",
  "gene_symbol": "MDN1",
  "gene_name": "Midasin"
}